{
  "gene_symbol": "IQCA1",
  "term_id": "GO:0005737",
  "gene": "UniProtKB:Q86XH1",
  "gene_name": "Dynein regulatory complex protein 11",
  "term_label": "cytoplasm"
}